{
  "gene_name": "Radical S-adenosyl methionine domain-containing protein 1, mitochondrial",
  "term_id": "GO:0006779",
  "term_label": "porphyrin-containing compound biosynthetic process",
  "gene": "UniProtKB:Q9HA92",
  "gene_symbol": "RSAD1"
}